{
  "gene_name": "Zinc finger protein 555",
  "term_label": "nucleus",
  "gene_symbol": "ZNF555",
  "gene": "UniProtKB:Q8NEP9",
  "term_id": "GO:0005634"
}